{
  "term_id": "GO:1990246",
  "gene": "UniProtKB:Q9NWR8",
  "gene_name": "Calcium uniporter regulatory subunit MCUb, mitochondrial",
  "gene_symbol": "MCUB",
  "term_label": "uniplex complex"
}